negative regulation of transport across blood-brain barrier [GO:0150202] (biological process) Relationships: is a type of negative regulation of transport [GO:0051051]; is a type of GO:0051241; is a type of regulation of transport across blood-brain barrier [GO:0150200]; BFO_0000050 negative regulation of vascular permeability [GO:0043116]; negatively regulates transport across blood-brain barrier [GO:0150104] Definition: Any process that stops, prevents or reduces the frequency, rate or extent of transport across blood-brain barrier. References: PMID:29377008, PMID:30280653 Sources: GOC:aruk, GOC:bc Subtypes: negative regulation of lipid transport across blood-brain barrier [GO:1903001]